{
  "gene_symbol": "ZC3H12D",
  "term_label": "mRNA binding",
  "term_id": "GO:0003729",
  "gene": "UniProtKB:A2A288",
  "gene_name": "Probable ribonuclease ZC3H12D"
}